{
  "term_id": "GO:1990782",
  "term_label": "protein tyrosine kinase binding",
  "gene_name": "Carcinoembryonic antigen-related cell adhesion molecule 20",
  "gene": "UniProtKB:Q6UY09",
  "gene_symbol": "CEACAM20"
}